{
  "gene": "UniProtKB:P62306",
  "term_label": "U1 snRNP",
  "gene_name": "Small nuclear ribonucleoprotein F",
  "term_id": "GO:0005685",
  "gene_symbol": "SNRPF"
}